{
  "gene_symbol": "COL14A1",
  "term_id": "GO:0005614",
  "gene_name": "Collagen alpha-1(XIV) chain",
  "gene": "UniProtKB:Q05707",
  "term_label": "interstitial matrix"
}